regulation of amino acid import across plasma membrane [GO:0010958] (biological process) Relationships: is_a regulation of amino acid transmembrane transport [GO:1903789]; regulates GO:0089718 Sources: GOC:dph, GOC:tb Definition: Any process that modulates the frequency, rate or extent of amino acid import into a cell. Subtypes: GO:0002036, regulation of D-aspartate import across plasma membrane [GO:0140215], regulation of glycine import across plasma membrane [GO:1900923], regulation of L-threonine import across plasma membrane [GO:1900926], regulation of L-tyrosine import across plasma membrane [GO:1900929], regulation of L-glutamine import across plasma membrane [GO:1901034], GO:1902834, regulation of L-lysine import across plasma membrane [GO:1905008], regulation of L-leucine import across plasma membrane [GO:1905532], GO:1905541, regulation of L-methionine import across plasma membrane [GO:1905624] Also known as: regulation of amino acid import